{
  "gene_name": "Probable G-protein coupled receptor 32",
  "term_id": "GO:0005886",
  "gene": "UniProtKB:O75388",
  "term_label": "plasma membrane",
  "gene_symbol": "GPR32"
}